{
  "term_id": "GO:0043235",
  "gene": "UniProtKB:P09619",
  "gene_name": "Platelet-derived growth factor receptor beta",
  "gene_symbol": "PDGFRB",
  "term_label": "receptor complex"
}